{
  "term_label": "membrane",
  "gene": "UniProtKB:Q6P1A2",
  "gene_name": "Lysophospholipid acyltransferase 5",
  "gene_symbol": "LPCAT3",
  "term_id": "GO:0016020"
}